{
  "gene_name": "Magnesium transporter NIPA1",
  "gene": "UniProtKB:Q7RTP0",
  "term_id": "GO:0015693",
  "gene_symbol": "NIPA1",
  "term_label": "magnesium ion transport"
}